{
  "term_label": "late endosome to vacuole transport via multivesicular body sorting pathway",
  "gene_symbol": "CHMP4BP1",
  "term_id": "GO:0032511",
  "gene_name": "Putative charged multivesicular body protein 4B-like protein CHMP4BP1",
  "gene": "UniProtKB:P59074"
}